{
  "term_id": "GO:0051233",
  "gene_symbol": "AURKC",
  "gene": "UniProtKB:Q9UQB9",
  "term_label": "spindle midzone",
  "gene_name": "Aurora kinase C"
}